negative regulation of endothelial cell proliferation [GO:0001937] (biological process) Relationships: is a type of GO:0001936; is a type of negative regulation of epithelial cell proliferation [GO:0050680]; RO_0002212 endothelial cell proliferation [GO:0001935] Sources: GOC:add Subtypes: GO:1903588, negative regulation of vascular endothelial cell proliferation [GO:1905563] Also known as: down regulation of endothelial cell proliferation, down-regulation of endothelial cell proliferation, downregulation of endothelial cell proliferation, inhibition of endothelial cell proliferation Definition: Any process that stops, prevents, or reduces the rate or extent of endothelial cell proliferation.